{
  "gene_symbol": "TMSB4X",
  "term_id": "GO:0003785",
  "gene_name": "Thymosin beta-4",
  "term_label": "actin monomer binding",
  "gene": "UniProtKB:P62328"
}